{
  "term_id": "GO:0005829",
  "gene": "UniProtKB:Q8IY22",
  "term_label": "cytosol",
  "gene_name": "C-Maf-inducing protein",
  "gene_symbol": "CMIP"
}